{
  "term_label": "Unknown cellular component",
  "gene_symbol": "FAM157C",
  "term_id": "UNKNOWN:0003",
  "gene_name": "Putative protein FAM157C",
  "gene": "UniProtKB:P0CG43"
}